{
  "gene_symbol": "PCDHGB4",
  "gene_name": "Protocadherin gamma-B4",
  "term_label": "cell adhesion",
  "gene": "UniProtKB:Q9UN71",
  "term_id": "GO:0007155"
}